negative regulation of signaling [GO:0023057] (biological process) Definition: Any process that stops, prevents, or reduces the frequency, rate or extent of a signaling process. Relationships: is a type of regulation of signaling [GO:0023051]; is a type of negative regulation of biological process [GO:0048519]; negatively regulates signaling [GO:0023052] Also known as: negative regulation of signaling process, negative regulation of signalling process Subtypes: GO:0001920, negative regulation of signal transduction [GO:0009968], negative regulation of hormone secretion [GO:0046888], GO:0050805, negative regulation of Wnt protein secretion [GO:0061358], negative regulation of c-di-GMP signaling [GO:0061942], negative regulation of trichome patterning [GO:1900033], GO:1905433, negative regulation of BMP secretion [GO:2001285] Sources: GOC:mtg_signal